{
  "term_id": "GO:0097524",
  "term_label": "sperm plasma membrane",
  "gene": "UniProtKB:P08910",
  "gene_symbol": "ABHD2",
  "gene_name": "Monoacylglycerol lipase ABHD2"
}